{
  "term_label": "G1/S transition of mitotic cell cycle",
  "gene": "UniProtKB:P20248",
  "gene_symbol": "CCNA2",
  "term_id": "GO:0000082",
  "gene_name": "Cyclin-A2"
}